{
  "gene_symbol": "ZNF160",
  "term_id": "GO:0005634",
  "gene_name": "Zinc finger protein 160",
  "gene": "UniProtKB:Q9HCG1",
  "term_label": "nucleus"
}